{
  "gene_symbol": "HPSE",
  "gene_name": "Heparanase",
  "term_id": "GO:0060055",
  "gene": "UniProtKB:Q9Y251",
  "term_label": "angiogenesis involved in wound healing"
}